{
  "gene": "UniProtKB:Q6YI46",
  "gene_name": "Transmembrane protein 64",
  "term_id": "GO:0045780",
  "gene_symbol": "TMEM64",
  "term_label": "positive regulation of bone resorption"
}